{
  "gene": "UniProtKB:Q9UI14",
  "gene_symbol": "RABAC1",
  "term_label": "Golgi apparatus",
  "gene_name": "Prenylated Rab acceptor protein 1",
  "term_id": "GO:0005794"
}